{
  "gene_symbol": "USP17L20",
  "gene": "UniProtKB:D6RJB6",
  "gene_name": "Ubiquitin carboxyl-terminal hydrolase 17-like protein 20",
  "term_id": "GO:0004843",
  "term_label": "cysteine-type deubiquitinase activity"
}